{
  "gene_name": "Ras-related protein Rab-11A",
  "gene_symbol": "RAB11A",
  "term_id": "GO:0006887",
  "term_label": "exocytosis",
  "gene": "UniProtKB:P62491"
}